{
  "gene_name": "Spindlin-2A",
  "term_id": "GO:0006355",
  "gene": "UniProtKB:Q99865",
  "gene_symbol": "SPIN2A",
  "term_label": "regulation of DNA-templated transcription"
}